{
  "gene_symbol": "SLC50A1",
  "term_id": "GO:0016020",
  "term_label": "membrane",
  "gene": "UniProtKB:Q9BRV3",
  "gene_name": "Sugar transporter SWEET1"
}